{
  "gene_symbol": "RTF2",
  "gene_name": "Replication termination factor 2",
  "term_id": "UNKNOWN:0001",
  "term_label": "Unknown molecular function",
  "gene": "UniProtKB:Q9BY42"
}